{
  "term_label": "cytoplasm",
  "gene_name": "Pyrin",
  "gene": "UniProtKB:O15553",
  "gene_symbol": "MEFV",
  "term_id": "GO:0005737"
}